{
  "gene_symbol": "DLGAP3",
  "term_label": "postsynaptic specialization",
  "gene": "UniProtKB:O95886",
  "gene_name": "Disks large-associated protein 3",
  "term_id": "GO:0099572"
}